{
  "gene_symbol": "CGAS",
  "gene_name": "Cyclic GMP-AMP synthase",
  "term_label": "2',3'-cyclic GMP-AMP synthase activity",
  "term_id": "GO:0061501",
  "gene": "UniProtKB:Q8N884"
}